cellular response to molecule of oomycetes origin [GO:0071227] (BP) Definition: Any process that results in a change in state or activity of a cell (in terms of movement, secretion, enzyme production, gene expression, etc.) as a result of a stimulus by molecules of oomycetes origin. Sources: GOC:mah Also known as: cellular response to oomycetes associated molecule Relationships: is a type of response to molecule of oomycetes origin [GO:0002240]; is_a cellular response to biotic stimulus [GO:0071216]; is part of response to fungus [GO:0009620]